{
  "gene_name": "Zinc finger protein 493",
  "term_label": "regulation of transcription by RNA polymerase II",
  "gene": "UniProtKB:Q6ZR52",
  "term_id": "GO:0006357",
  "gene_symbol": "ZNF493"
}